{
  "term_id": "GO:0005615",
  "term_label": "extracellular space",
  "gene": "UniProtKB:P02808",
  "gene_symbol": "STATH",
  "gene_name": "Statherin"
}